cardiac muscle contraction [GO:0060048] (biological process) Also known as: heart muscle contraction Definition: Muscle contraction of cardiac muscle tissue. Relationships: is a type of striated muscle contraction [GO:0006941]; is part of heart contraction [GO:0060047] Sources: GOC:dph Regulation: regulated by regulation of cardiac muscle contraction [GO:0055117]; negatively regulated by negative regulation of cardiac muscle contraction [GO:0055118]; positively regulated by positive regulation of cardiac muscle contraction [GO:0060452]